{
  "term_id": "UNKNOWN:0002",
  "term_label": "Unknown biological process",
  "gene_name": "Protein phosphatase 1 regulatory subunit 16A",
  "gene": "UniProtKB:Q96I34",
  "gene_symbol": "PPP1R16A"
}